{
  "gene": "UniProtKB:Q9BYW3",
  "gene_symbol": "DEFB126",
  "gene_name": "Beta-defensin 126",
  "term_label": "Unknown cellular component",
  "term_id": "UNKNOWN:0003"
}